{
  "term_label": "phosphatidic acid binding",
  "gene_name": "Pleckstrin homology domain-containing family N member 1",
  "gene_symbol": "PLEKHN1",
  "term_id": "GO:0070300",
  "gene": "UniProtKB:Q494U1"
}